{
  "gene_name": "Dual specificity protein phosphatase 16",
  "term_id": "GO:0008330",
  "term_label": "protein tyrosine/threonine phosphatase activity",
  "gene_symbol": "DUSP16",
  "gene": "UniProtKB:Q9BY84"
}